{
  "term_id": "GO:0005886",
  "gene": "UniProtKB:O60928",
  "term_label": "plasma membrane",
  "gene_name": "Inward rectifier potassium channel 13",
  "gene_symbol": "KCNJ13"
}